RNA-directed RNA polymerase activity [GO:0003968] (molecular function) Definition: Catalysis of the reaction: nucleoside triphosphate + RNA(n) = diphosphate + RNA(n+1); uses an RNA template, i.e. the catalysis of RNA-template-directed extension of the 3'-end of an RNA strand by one nucleotide at a time. Relationships: is a type of 5'-3' RNA polymerase activity [GO:0034062]; is part of RNA-templated transcription [GO:0001172] Also known as: transcriptase, RNA nucleotidyltransferase (RNA-directed) activity, RNA-dependent RNA polymerase activity, RNA-dependent RNA replicase activity, RNA-directed 5'-3' RNA polymerase activity, RdRP activity, RNA replicase activity, RNA synthetase activity Sources: EC:2.7.7.48, GOC:mah, GOC:pf Regulation: RO_0002212 by negative regulation of RNA-dependent RNA polymerase activity [GO:1900260]